{
  "gene_symbol": "PRF1",
  "gene": "UniProtKB:P14222",
  "gene_name": "Perforin-1",
  "term_id": "GO:0002357",
  "term_label": "defense response to tumor cell"
}